{
  "term_label": "centrosome",
  "gene": "UniProtKB:P41208",
  "gene_symbol": "CETN2",
  "term_id": "GO:0005813",
  "gene_name": "Centrin-2"
}